trigeminal sensory nucleus development [GO:0021730] (biological process) Subtypes: mesencephalic trigeminal nucleus development [GO:0021739], principal sensory nucleus of trigeminal nerve development [GO:0021740], spinal trigeminal nucleus development [GO:0021741] Note: Note that this term was placed as a child of 'brain development' because the nucleus spans multiple brain regions from midbrain to spinal cord. Sources: GOC:cls, GOC:curators, GOC:dgh, GOC:dph, GOC:jid Relationships: is a type of neural nucleus development [GO:0048857]; is part of brain development [GO:0007420] Definition: The process whose specific outcome is the progression of the trigeminal sensory nucleus over time, from its formation to the mature structure.